{
  "gene": "UniProtKB:Q9NS00",
  "term_id": "GO:0016263",
  "gene_symbol": "C1GALT1",
  "term_label": "glycoprotein-N-acetylgalactosamine 3-beta-galactosyltransferase activity",
  "gene_name": "Glycoprotein-N-acetylgalactosamine 3-beta-galactosyltransferase 1"
}